{
  "term_label": "transcription cis-regulatory region binding",
  "gene": "UniProtKB:Q9UK10",
  "term_id": "GO:0000976",
  "gene_symbol": "ZNF225",
  "gene_name": "Zinc finger protein 225"
}